{
  "gene": "UniProtKB:Q9UBD3",
  "term_id": "GO:0030335",
  "gene_symbol": "XCL2",
  "term_label": "positive regulation of cell migration",
  "gene_name": "Cytokine SCM-1 beta"
}